proximal portion of axoneme [GO:0120134] (cellular component) Definition: The portion of the axoneme that is close to the base of the cilium. Sources: GOC:krc Relationships: is a type of cellular anatomical structure [GO:0110165]; is part of axoneme [GO:0005930] Also known as: proximal part of axoneme